{
  "gene_symbol": "PRPS1L1",
  "gene_name": "Ribose-phosphate pyrophosphokinase 3",
  "term_id": "GO:0006164",
  "term_label": "purine nucleotide biosynthetic process",
  "gene": "UniProtKB:P21108"
}